{
  "term_id": "UNKNOWN:0002",
  "term_label": "Unknown biological process",
  "gene_name": "Dehydrogenase_reductase SDR family member 7B",
  "gene": "UniProtKB:Q6IAN0",
  "gene_symbol": "DHRS7B"
}